{
  "gene_symbol": "SNAPC2",
  "gene": "UniProtKB:Q13487",
  "term_label": "Unknown molecular function",
  "term_id": "UNKNOWN:0001",
  "gene_name": "snRNA-activating protein complex subunit 2"
}